{
  "gene_name": "Exostosin-like 3",
  "gene_symbol": "EXTL3",
  "term_label": "glycosyltransferase activity",
  "gene": "UniProtKB:O43909",
  "term_id": "GO:0016757"
}